{
  "term_label": "cytosol",
  "term_id": "GO:0005829",
  "gene": "UniProtKB:Q9H0C5",
  "gene_name": "BTB_POZ domain-containing protein 1",
  "gene_symbol": "BTBD1"
}